{
  "gene_name": "Protein FAM8A1",
  "gene_symbol": "FAM8A1",
  "term_label": "Unknown cellular component",
  "gene": "UniProtKB:Q9UBU6",
  "term_id": "UNKNOWN:0003"
}